{
  "gene": "UniProtKB:Q9UN81",
  "term_id": "GO:1990904",
  "gene_name": "LINE-1 retrotransposable element ORF1 protein",
  "term_label": "ribonucleoprotein complex",
  "gene_symbol": "L1RE1"
}